{
  "gene_symbol": "FASTKD1",
  "term_label": "mitochondrial RNA processing",
  "gene_name": "FAST kinase domain-containing protein 1, mitochondrial",
  "term_id": "GO:0000963",
  "gene": "UniProtKB:Q53R41"
}